{
  "gene": "UniProtKB:Q99707",
  "gene_name": "Methionine synthase",
  "term_id": "GO:0008705",
  "term_label": "methionine synthase activity",
  "gene_symbol": "MTR"
}